procollagen-proline 4-dioxygenase activity [GO:0004656] (molecular function) Definition: Catalysis of the reaction: procollagen L-proline + 2-oxoglutarate + O2 = procollagen trans-4-hydroxy-L-proline + succinate + CO2. Also known as: peptidyl proline hydroxylase activity, proline hydroxylase activity, proline, 2-oxoglutarate dioxygenase activity, proline,2-oxoglutarate 4-dioxygenase activity, prolyl 4-hydroxylase activity, prolyl hydroxylase activity, prolyl-glycyl-peptide, 2-oxoglutarate:oxygen oxidoreductase, 4-hydroxylating activity, protocollagen hydroxylase activity, procollagen-proline,2-oxoglutarate-4-dioxygenase activity, collagen proline hydroxylase activity, hydroxylase, collagen proline activity, procollagen-L-proline,2-oxoglutarate:oxygen oxidoreductase (4-hydroxylating) activity, proline protocollagen hydroxylase activity, prolylprotocollagen dioxygenase activity, prolylprotocollagen hydroxylase activity, protocollagen proline 4-hydroxylase activity, protocollagen proline dioxygenase activity, protocollagen proline hydroxylase activity, protocollagen prolyl hydroxylase activity Relationships: is a type of procollagen-proline dioxygenase activity [GO:0019798]; is a type of peptidyl-proline 4-dioxygenase activity [GO:0031545] Sources: EC:1.14.11.2